alcohol dehydrogenase (cytochrome c(L)) activity [GO:0052933] (molecular function) Definition: Catalysis of the reaction: 2 [Fe(III)cytochrome cL] + a primary alcohol = 2 [Fe(II)cytochrome cL] + an aldehyde + 2 H+. Sources: RHEA:51004 Also known as: alcohol:cytochrome c(L) oxidoreductase activity, 2-chloroethanol cytochrome-c oxidoreductase activity, ethanol cytochrome-c oxidoreductase activity, methanol dehydrogenase activity, methanol ferricytochrome-c oxidoreductase activity Relationships: is a type of GO:0016898